{
  "term_id": "UNKNOWN:0002",
  "gene_name": "Peptidase inhibitor R3HDML",
  "gene": "UniProtKB:Q9H3Y0",
  "term_label": "Unknown biological process",
  "gene_symbol": "R3HDML"
}